inositol 4-methyltransferase activity [GO:0030787] (molecular function) Definition: Catalysis of the reaction: S-adenosyl-L-methionine(1+) + myo-inositol = 1D-4-O-methyl-myo-inositol + S-adenosyl-L-homocysteine + H+. Relationships: is a type of GO:0008757 Also known as: S-adenosyl-L-methionine:1D-myo-inositol 4-methyltransferase activity, S-adenosyl-L-methionine:myo-inositol 4-O-methyltransferase activity, myo-inositol 4-O-methyltransferase activity, myo-inositol 6-O-methyltransferase activity Sources: EC:2.1.1.129, RHEA:23248